{
  "term_label": "cytoplasm",
  "gene": "UniProtKB:Q6UUV9",
  "term_id": "GO:0005737",
  "gene_symbol": "CRTC1",
  "gene_name": "CREB-regulated transcription coactivator 1"
}